chondroitin sulfate proteoglycan biosynthetic process [GO:0050650] (biological process) Also known as: chondroitin sulfate proteoglycan anabolism, chondroitin sulfate proteoglycan biosynthesis, chondroitin sulfate proteoglycan formation, chondroitin sulfate proteoglycan synthesis, chondroitin sulphate proteoglycan biosynthesis, chondroitin sulphate proteoglycan biosynthetic process References: PMID:17239763 Relationships: is a type of proteoglycan biosynthetic process [GO:0030166]; is a type of chondroitin sulfate proteoglycan metabolic process [GO:0050654]; is a type of GO:0180064 Definition: The chemical reactions and pathways resulting in the formation of chondroitin sulfate proteoglycans, which consist of a core protein linked to a chondroitin sulfate glycosaminoglycan. The chondroitin sulfate chain is composed of the repeating disaccharide unit beta-(1,4)-D-glucuronic acid-beta-(1,3)-N-acetyl-D-galactosamine, the latter of which can be O-sulfated. Chondroitin sulfate chains are covalently linked to serine/threonine residues (O-linked) of the core protein via a tetrasaccharide linker sequence (xylose-galactose-galactose-glucuronate).